{
  "gene_symbol": "MED13L",
  "gene_name": "Mediator of RNA polymerase II transcription subunit 13-like",
  "term_label": "Unknown cellular component",
  "term_id": "UNKNOWN:0003",
  "gene": "UniProtKB:Q71F56"
}